tau-protein kinase activity [GO:0050321] (molecular function) Sources: EC:2.7.11.26 Definition: Catalysis of the reaction: ATP + tau-protein = ADP + O-phospho-tau-protein on serine and threonine residues. Relationships: is a type of GO:0004674 Also known as: ATP:tau-protein O-phosphotransferase activity, [Tau protein] kinase activity, brain protein kinase PK40erk activity, tau-protein kinase I activity, tau-protein kinase II activity, tau-tubulin kinase activity, CDK5/p23, GSK, STK31, TPK, TPK I, TPK II, TTK, cdk5/p20, glycogen synthase kinase-3beta activity, protein tau kinase activity, tau kinase activity, tau protein kinase activity